{
  "term_id": "GO:0045271",
  "gene_name": "NADH dehydrogenase [ubiquinone] iron-sulfur protein 2, mitochondrial",
  "gene": "UniProtKB:O75306",
  "term_label": "respiratory chain complex I",
  "gene_symbol": "NDUFS2"
}